{
  "term_label": "alpha DNA polymerase:primase complex",
  "term_id": "GO:0005658",
  "gene_name": "DNA primase small subunit",
  "gene_symbol": "PRIM1",
  "gene": "UniProtKB:P49642"
}